octopamine metabolic process [GO:0046333] (biological process) Relationships: is a type of GO:0006066; is a type of GO:0018958 Subtypes: GO:0006589, GO:0046334 Sources: ISBN:0198506732 Also known as: octopamine metabolism Definition: The chemical reactions and pathways involving octopamine, 1-(p-hydroxyphenyl)-2-aminoethanol. The D enantiomer is about one-tenth as active as norepinephrine and is found in the salivary glands of Octopus and Eledone species.